{
  "term_id": "GO:0032783",
  "gene_name": "AF4_FMR2 family member 3",
  "gene": "UniProtKB:P51826",
  "term_label": "super elongation complex",
  "gene_symbol": "AFF3"
}